mitochondrial intracristal space [GO:0044290] (cellular component) Sources: NIF_Subcellular:sao508958414 Relationships: is a type of cellular anatomical structure [GO:0110165]; is part of mitochondrion [GO:0005739] Definition: The space bounded by the mitochondrial cristae membranes, continuous with the intermembrane space.